{
  "gene": "UniProtKB:P08218",
  "term_label": "serine-type endopeptidase activity",
  "gene_name": "Chymotrypsin-like elastase family member 2B",
  "gene_symbol": "CELA2B",
  "term_id": "GO:0004252"
}